{
  "gene_name": "Myomesin-1",
  "gene_symbol": "MYOM1",
  "term_label": "structural constituent of muscle",
  "term_id": "GO:0008307",
  "gene": "UniProtKB:P52179"
}